extracellular exosome [GO:0070062] (cellular component) References: PMID:15908444, PMID:17641064, PMID:19442504, PMID:19498381, PMID:22418571, PMID:24009894 Sources: GOC:BHF, GOC:mah, GOC:vesicles Relationships: is a type of extracellular vesicle [GO:1903561]; is part of extracellular space [GO:0005615] Also known as: exosome, extracellular vesicular exosome Definition: A vesicle that is released into the extracellular region by fusion of the limiting endosomal membrane of a multivesicular body with the plasma membrane. Extracellular exosomes, also simply called exosomes, have a diameter of about 40-100 nm.